regulation of aeciospore formation [GO:0075248] (biological process) Subtypes: positive regulation of aeciospore formation [GO:0075249], GO:0075250 Relationships: is a type of GO:0043943; regulates aeciospore formation [GO:0075247] Definition: Any process that modulates the frequency, rate or extent of aeciospore formation, a process in which a dikaryotic spore of typically a rust fungus is produced in an aecium. Sources: GOC:pamgo_curators